DNA 5-methylcytosine dioxygenase activity [GO:0070579] (molecular function) References: PMID:19372391, PMID:21496894, PMID:21778364 Sources: EC:1.14.11.80 Also known as: methylcytosine dioxygenase activity Note: This reaction removes the methyl group from position 5 of cytosine in DNA via oxidation of the 5-methylcytosine, followed by removal of the oxidised base by the base excision repair system. Do not confuse with oxidative DNA demethylase activity ; GO:0035516, which directly reverses the alkylation on nucleotides in the DNA. Relationships: is a type of 2-oxoglutarate-dependent dioxygenase activity [GO:0016706]; is a type of GO:0140097 Definition: Catalysis of the reaction: 5-methylcytosine (5mC) in DNA + 2-oxoglutarate + O2 = 5-hydroxymethylcytosine (5hmC) in DNA + succinate + CO2. This reaction is the first step in the removal of cytosine methylated on position 5 in double-stranded DNA. This activity can iteratively oxidize 5hmC to 5-formylcytosine (5fC) and to 5-carboxylcytosine (5caC).